acetate CoA-transferase complex [GO:0009329] (cellular component) Subtypes: GO:0032283 References: PMID:2719476, PMID:8423010 Sources: GOC:jl Relationships: is_a transferase complex [GO:1990234]; is part of acetyl-CoA carboxylase complex [GO:0009317] Definition: A heterotetrameric enzyme complex made up of two alpha subunits and two beta subunits. Part of the acetyl-CoA carboxylase complex. Catalyzes the transfer of a carboxyl group to form malonyl-CoA.